{
  "gene": "UniProtKB:Q6P656",
  "gene_name": "Cilia- and flagella-associated protein 161",
  "gene_symbol": "CFAP161",
  "term_label": "Unknown molecular function",
  "term_id": "UNKNOWN:0001"
}